{
  "term_id": "GO:0016020",
  "gene_symbol": "RABIF",
  "term_label": "membrane",
  "gene_name": "Guanine nucleotide exchange factor MSS4",
  "gene": "UniProtKB:P47224"
}